{
  "term_id": "GO:0005890",
  "gene_name": "Sodium_potassium-transporting ATPase subunit alpha-4",
  "gene": "UniProtKB:Q13733",
  "gene_symbol": "ATP1A4",
  "term_label": "sodium:potassium-exchanging ATPase complex"
}